positive regulation of granuloma formation [GO:0002633] (biological process) Sources: GOC:add Definition: Any process that activates or increases the frequency, rate, or extent of granuloma formation. Also known as: up regulation of granuloma formation, up-regulation of granuloma formation, upregulation of granuloma formation, activation of granuloma formation, stimulation of granuloma formation Relationships: is a type of GO:0002631; is a type of positive regulation of chronic inflammatory response [GO:0002678]; is a type of GO:0002699; positively regulates granuloma formation [GO:0002432]